{
  "term_id": "GO:0060339",
  "gene": "UniProtKB:Q86WI3",
  "gene_symbol": "NLRC5",
  "term_label": "negative regulation of type I interferon-mediated signaling pathway",
  "gene_name": "Protein NLRC5"
}